venom-mediated vasodilation [GO:0044551] (biological process) Definition: A process in which an organism initiates, promotes, or enhances the widening of blood vessels by small muscles in their walls in another organism via the action of a venom, concomittantly reducing blood pressure in the bitten/stung organism. Subtypes: GO:0140162, venom-mediated vasodilation by activation of nitric oxide-cGMP-mediated signaling [GO:0140165], venom-mediated vasodilation via suppression of angiotensin maturation [GO:0140166] Also known as: envenomation resulting in vasodilation in another organism, envenomation resulting in vasodilation in other organism, venom-mediated vasorelaxation, envenomation resulting in modulation of vasodilation in other organism, envenomation resulting in regulation of vasodilation in other organism References: PMID:21050868 Sources: GOC:ecd, GOC:jl Relationships: is a type of venom-mediated perturbation of blood circulation [GO:0140134]